{
  "gene_name": "Uncharacterized protein C17orf78",
  "term_label": "Unknown cellular component",
  "gene_symbol": "C17orf78",
  "term_id": "UNKNOWN:0003",
  "gene": "UniProtKB:Q8N4C9"
}